{
  "term_id": "GO:0007224",
  "term_label": "smoothened signaling pathway",
  "gene_name": "Protein dispatched homolog 2",
  "gene": "UniProtKB:A7MBM2",
  "gene_symbol": "DISP2"
}